{
  "term_label": "3',5'-cyclic-GMP phosphodiesterase activity",
  "gene_name": "Rod cGMP-specific 3',5'-cyclic phosphodiesterase subunit alpha",
  "term_id": "GO:0047555",
  "gene_symbol": "PDE6A",
  "gene": "UniProtKB:P16499"
}